regulation of CD8-positive, alpha-beta T cell differentiation [GO:0043376] (biological process) Definition: Any process that modulates the frequency, rate, or extent of CD8-positive, alpha-beta T cell differentiation. Sources: GOC:add, ISBN:0781735149 Also known as: regulation of CD8-positive T lymphocyte differentiation, regulation of CD8-positive T-cell differentiation, regulation of CD8-positive T-lymphocyte differentiation, regulation of CD8-positive, alpha beta T lymphocyte differentiation, regulation of CD8-positive, alpha beta T-cell differentiation, regulation of CD8-positive, alpha beta T-lymphocyte differentiation, regulation of CD8-positive, alpha-beta T cell development Note: Note that immunologists typically use the word 'development' to refer to cells of B or T cell lineages undergoing the process that GO describes as 'cell differentiation'. Relationships: is_a regulation of alpha-beta T cell differentiation [GO:0046637]; is_a regulation of CD8-positive, alpha-beta T cell activation [GO:2001185]; regulates GO:0043374 Subtypes: negative regulation of CD8-positive, alpha-beta T cell differentiation [GO:0043377], positive regulation of CD8-positive, alpha-beta T cell differentiation [GO:0043378]